{
  "term_label": "uniplex complex",
  "term_id": "GO:1990246",
  "gene": "UniProtKB:Q8NE86",
  "gene_symbol": "MCU",
  "gene_name": "Calcium uniporter protein, mitochondrial"
}